{
  "term_id": "UNKNOWN:0003",
  "gene_name": "Pregnancy-specific beta-1-glycoprotein 4",
  "gene_symbol": "PSG4",
  "term_label": "Unknown cellular component",
  "gene": "UniProtKB:Q00888"
}